{
  "term_label": "response to exogenous dsRNA",
  "gene_name": "Interferon alpha-4",
  "gene": "UniProtKB:P05014",
  "term_id": "GO:0043330",
  "gene_symbol": "IFNA4"
}